{
  "term_id": "UNKNOWN:0002",
  "term_label": "Unknown biological process",
  "gene_symbol": "AGBL2",
  "gene": "UniProtKB:Q5U5Z8",
  "gene_name": "Cytosolic carboxypeptidase 2"
}